{
  "gene_symbol": "NR1H2",
  "gene_name": "Oxysterols receptor LXR-beta",
  "gene": "UniProtKB:P55055",
  "term_label": "nucleus",
  "term_id": "GO:0005634"
}